{
  "term_label": "endoplasmic reticulum tubular network formation",
  "gene": "UniProtKB:O75298",
  "term_id": "GO:0071787",
  "gene_name": "Reticulon-2",
  "gene_symbol": "RTN2"
}